{
  "term_id": "GO:0000149",
  "term_label": "SNARE binding",
  "gene": "UniProtKB:Q7Z7G2",
  "gene_symbol": "CPLX4",
  "gene_name": "Complexin-4"
}